protein-N(PI)-phosphohistidine-sorbitol phosphotransferase system transporter activity [GO:0022856] (molecular function) Relationships: is a type of protein-N(PI)-phosphohistidine-sugar phosphotransferase activity [GO:0008982]; is a type of GO:0015576 Sources: GOC:mtg_transport, ISBN:0815340729 Also known as: sorbitol PTS transporter activity Definition: Catalysis of the PEP-dependent, phosphoryl transfer-driven transport of substances across a membrane. The transport happens by catalysis of the reaction: protein N-phosphohistidine + sorbitol(out) = protein histidine + sorbitol phosphate(in). This differs from primary and secondary active transport in that the solute is modified during transport.